{
  "gene_name": "Transmembrane protein 14EP",
  "term_label": "Unknown molecular function",
  "term_id": "UNKNOWN:0001",
  "gene_symbol": "TMEM14EP",
  "gene": "UniProtKB:Q6UXP3"
}